{
  "gene_name": "Dynactin subunit 3",
  "gene": "UniProtKB:O75935",
  "gene_symbol": "DCTN3",
  "term_label": "dynactin complex",
  "term_id": "GO:0005869"
}